{
  "term_id": "GO:0005634",
  "gene": "UniProtKB:P78415",
  "gene_name": "Iroquois-class homeodomain protein IRX-3",
  "term_label": "nucleus",
  "gene_symbol": "IRX3"
}